{
  "gene_name": "Interferon-stimulated gene 20 kDa protein",
  "gene_symbol": "ISG20",
  "gene": "UniProtKB:Q96AZ6",
  "term_label": "RNA catabolic process",
  "term_id": "GO:0006401"
}